fructose-bisphosphate aldolase activity [GO:0004332] (molecular function) Definition: Catalysis of the reaction: beta-D-fructose 1,6-bisphosphate = D-glyceraldehyde 3-phosphate + dihydroxyacetone phosphate. Relationships: is a type of aldehyde-lyase activity [GO:0016832] Also known as: aldolase activity, 1,6-diphosphofructose aldolase activity, D-fructose-1,6-bisphosphate D-glyceraldehyde-3-phosphate-lyase (glycerone-phosphate-forming), D-fructose-1,6-bisphosphate D-glyceraldehyde-3-phosphate-lyase activity, SMALDO, diphosphofructose aldolase activity, fructoaldolase activity, fructose 1,6-diphosphate aldolase activity, fructose 1-monophosphate aldolase activity, fructose 1-phosphate aldolase activity, fructose diphosphate aldolase activity, fructose-1,6-bisphosphate triosephosphate-lyase activity, ketose 1-phosphate aldolase activity, phosphofructoaldolase activity, zymohexase activity Sources: EC:4.1.2.13